{
  "gene": "UniProtKB:A6NFY4",
  "term_id": "UNKNOWN:0002",
  "term_label": "Unknown biological process",
  "gene_name": "Nuclear envelope integral membrane protein 2",
  "gene_symbol": "NEMP2"
}